{
  "term_id": "GO:0007507",
  "term_label": "heart development",
  "gene_name": "Transcription factor SOX-9",
  "gene_symbol": "SOX9",
  "gene": "UniProtKB:P48436"
}